thiamine salvage [GO:0036172] (biological process) Definition: A process that generates thiamine (vitamin B1) from derivatives of it without de novo synthesis. References: PMID:15150256, PMID:16952958 Relationships: is a type of pyrimidine-containing compound salvage [GO:0008655]; is_a thiamine biosynthetic process [GO:0009228]